synaptobrevin 2-SNAP-25-syntaxin-2 complex [GO:0070045] (cellular component) References: PMID:10336434 Relationships: is a type of SNARE complex [GO:0031201] Also known as: SNARE complex (Stx2, Snap25, Vamp2), Stx2-Snap25-Vamp2 complex Definition: A SNARE complex that contains synaptobrevin 2 (VAMP2), SNAP-25, and syntaxin 2 (or orthologs thereof).